{
  "gene": "UniProtKB:Q5VZ72",
  "gene_name": "Izumo sperm-egg fusion protein 3",
  "gene_symbol": "IZUMO3",
  "term_id": "UNKNOWN:0003",
  "term_label": "Unknown cellular component"
}